{
  "gene_symbol": "TNFSF12",
  "gene": "UniProtKB:O43508",
  "term_label": "extrinsic apoptotic signaling pathway",
  "gene_name": "Tumor necrosis factor ligand superfamily member 12",
  "term_id": "GO:0097191"
}